positive regulation of cell migration by VEGF-activated platelet derived growth factor receptor signaling pathway [GO:0038090] (biological process) References: PMID:17470632 Sources: GOC:bf, GOC:signaling Definition: The series of molecular signals initiated by vascular endothelial growth factor (VEGF) binding to a platelet-derived growth factor receptor (PDGFR) on the surface of a cell, which activates or increases the frequency, rate or extent of the orderly movement of a cell from one site to another. Also known as: VEGF/PDGFR-induced cell migration, positive regulation of cell migration by VEGF-activated platelet derived growth factor receptor signalling pathway, positive regulation of cell migration by VEGF/PDGFR signaling pathway Relationships: is a type of VEGF-activated platelet-derived growth factor receptor signaling pathway [GO:0038086]; is a type of positive regulation of cell migration by vascular endothelial growth factor signaling pathway [GO:0038089]